{
  "term_id": "GO:0005615",
  "gene_symbol": "BCAM",
  "term_label": "extracellular space",
  "gene_name": "Basal cell adhesion molecule",
  "gene": "UniProtKB:P50895"
}